{
  "gene": "UniProtKB:O75596",
  "term_label": "Unknown molecular function",
  "gene_symbol": "CLEC3A",
  "gene_name": "C-type lectin domain family 3 member A",
  "term_id": "UNKNOWN:0001"
}